{
  "gene_name": "Meteorin",
  "gene": "UniProtKB:Q9UJH8",
  "gene_symbol": "METRN",
  "term_id": "GO:0005615",
  "term_label": "extracellular space"
}